{
  "gene_symbol": "AGTRAP",
  "gene": "UniProtKB:Q6RW13",
  "term_id": "GO:0005886",
  "gene_name": "Type-1 angiotensin II receptor-associated protein",
  "term_label": "plasma membrane"
}